{
  "term_label": "actin filament binding",
  "gene": "UniProtKB:Q9H254",
  "gene_symbol": "SPTBN4",
  "term_id": "GO:0051015",
  "gene_name": "Spectrin beta chain, non-erythrocytic 4"
}